{
  "term_id": "GO:0003677",
  "term_label": "DNA binding",
  "gene_symbol": "TAF12",
  "gene": "UniProtKB:Q16514",
  "gene_name": "Transcription initiation factor TFIID subunit 12"
}